Sep-tRNA:Cys-tRNA synthase activity [GO:0043766] (molecular function) Relationships: is a type of transferase activity, transferring alkyl or aryl (other than methyl) groups [GO:0016765]; is a type of catalytic activity, acting on a tRNA [GO:0140101]; is part of conversion of O-phosphoseryl-tRNA to cysteinyl-tRNA [GO:0071952] References: PMID:15790858, PMID:16380427, PMID:17110438 Sources: RHEA:25686 Also known as: O-phosphoseryl-tRNA:cysteinyl-tRNA synthase activity, Sep-tRNA:Cys-tRNA synthetase activity, SepCysS Definition: Catalysis of the reaction: H+ + hydrogen sulfide + O-phospho-L-seryl-tRNA(Cys) = L-cysteinyl-tRNA(Cys) + phosphate.